{
  "gene_symbol": "RPS6KL1",
  "term_id": "UNKNOWN:0003",
  "term_label": "Unknown cellular component",
  "gene": "UniProtKB:Q9Y6S9",
  "gene_name": "Ribosomal protein S6 kinase-like 1"
}